{
  "term_label": "proteolysis",
  "gene_symbol": "ADAMTS1",
  "gene_name": "A disintegrin and metalloproteinase with thrombospondin motifs 1",
  "gene": "UniProtKB:Q9UHI8",
  "term_id": "GO:0006508"
}